{
  "gene_symbol": "ST8SIA5",
  "term_id": "GO:0006491",
  "gene_name": "Alpha-2,8-sialyltransferase 8E",
  "term_label": "N-glycan processing",
  "gene": "UniProtKB:O15466"
}